trunk neural crest cell migration [GO:0036484] (biological process) Also known as: trunk NCC migration Definition: The characteristic movement of trunk neural crest cells from the neural tube to other locations in the vertebrate embryo. Subtypes: GO:0036485, ventral trunk neural crest cell migration [GO:0036486] Relationships: is a type of neural crest cell migration [GO:0001755]; is part of GO:0035290 References: PMID:2387238 Sources: GOC:PARL, GOC:bf, GOC:mat